shelterin complex assembly [GO:0071573] (biological process) Definition: The aggregation, arrangement and bonding together of a set of components to form a shelterin complex. A shelterin complex is a nuclear telomere cap complex that is formed by the association of telomeric ssDNA- and dsDNA-binding proteins with telomeric DNA, and is involved in telomere protection and recruitment of telomerase. Regulation: RO_0002211 by GO:1904790; negatively regulated by negative regulation of shelterin complex assembly [GO:1904791]; positively regulated by positive regulation of shelterin complex assembly [GO:1904792] Sources: GOC:mah, GOC:vw Also known as: telosome assembly, Pot1 complex assembly, Pot1-Tpz1 complex assembly, shelterin complex formation Relationships: is a type of protein-DNA complex assembly [GO:0065004]; is part of GO:0032200